{
  "gene_symbol": "KCNJ15",
  "gene": "UniProtKB:Q99712",
  "gene_name": "ATP-sensitive inward rectifier potassium channel 15",
  "term_label": "inward rectifier potassium channel activity",
  "term_id": "GO:0005242"
}